negative regulation of cardiac ventricle development [GO:1904413] (biological process) Definition: Any process that stops, prevents or reduces the frequency, rate or extent of cardiac ventricle development. Also known as: down regulation of cardiac ventricle development, down-regulation of cardiac ventricle development, downregulation of cardiac ventricle development, inhibition of cardiac ventricle development References: PMID:19590510 Sources: GOC:TermGenie, GO_REF:0000058 Relationships: is a type of negative regulation of developmental process [GO:0051093]; is_a GO:0051241; is a type of regulation of cardiac ventricle development [GO:1904412]; negatively regulates cardiac ventricle development [GO:0003231] Subtypes: GO:1904943